{
  "term_id": "UNKNOWN:0003",
  "gene_name": "Zinc finger MYND domain-containing protein 12",
  "gene": "UniProtKB:Q9H0C1",
  "gene_symbol": "ZMYND12",
  "term_label": "Unknown cellular component"
}